{
  "gene_symbol": "PLCG2",
  "gene_name": "1-phosphatidylinositol 4,5-bisphosphate phosphodiesterase gamma-2",
  "term_label": "ruffle membrane",
  "term_id": "GO:0032587",
  "gene": "UniProtKB:P16885"
}